{
  "term_id": "GO:0007155",
  "gene_name": "Protocadherin alpha-4",
  "gene_symbol": "PCDHA4",
  "term_label": "cell adhesion",
  "gene": "UniProtKB:Q9UN74"
}